ABC-type D-ribose transporter activity [GO:0015611] (molecular function) Definition: Enables the transfer of a solute or solutes from one side of a membrane to the other according to the reaction: ATP + H2O + D-ribose(out) = ADP + phosphate + D-ribose(in). Also known as: D-ribose porter activity, D-ribose-importing ATPase activity Relationships: is a type of ABC-type monosaccharide transporter activity [GO:0015407]; is a type of GO:0015591 Sources: RHEA:29903